mitogen-activated protein kinase kinase binding [GO:0031434] (molecular function) Sources: GOC:mah Also known as: MAPKK binding Relationships: is a type of protein kinase binding [GO:0019901] Definition: Binding to a mitogen-activated protein kinase kinase, a protein that can phosphorylate a MAP kinase.